{
  "term_label": "plasma membrane",
  "gene_name": "Claudin-18",
  "gene": "UniProtKB:P56856",
  "gene_symbol": "CLDN18",
  "term_id": "GO:0005886"
}